{
  "gene_name": "ADP-ribosyl cyclase_cyclic ADP-ribose hydrolase 2",
  "term_label": "plasma membrane",
  "term_id": "GO:0005886",
  "gene": "UniProtKB:Q10588",
  "gene_symbol": "BST1"
}